{
  "term_label": "Unknown molecular function",
  "gene_symbol": "HAPSTR1",
  "term_id": "UNKNOWN:0001",
  "gene": "UniProtKB:Q14CZ0",
  "gene_name": "HUWE1-associated protein modifying stress responses 1"
}